{
  "gene_symbol": "NDUFV1-DT",
  "term_label": "Unknown biological process",
  "gene": "UniProtKB:Q8NBR9",
  "gene_name": "Uncharacterized protein NDUFV1-DT",
  "term_id": "UNKNOWN:0002"
}